regulation of response to nutrient levels [GO:0032107] (biological process) Definition: Any process that modulates the frequency, rate or extent of a response to nutrient levels. Relationships: is a type of regulation of response to stimulus [GO:0048583]; regulates GO:0031667 Sources: GOC:mah Subtypes: GO:0006792, regulation of nitrogen utilization [GO:0006808], regulation of response to food [GO:0032095], negative regulation of response to nutrient levels [GO:0032108], positive regulation of response to nutrient levels [GO:0032109], regulation of carbon utilization [GO:0043609], regulation of carbohydrate utilization [GO:0043610], regulation of aggregation involved in sorocarp development [GO:0060176], GO:0060905, regulation of vitamin D receptor signaling pathway [GO:0070562], regulation of cellular response to phosphate starvation [GO:0140255], regulation of filamentous growth of a population of unicellular organisms in response to starvation [GO:1900434], regulation of cellular response to iron ion starvation [GO:1901966], regulation of cellular response to amino acid starvation [GO:1903832], GO:1904547